RNA stabilization [GO:0043489] (biological process) Sources: GOC:go_curators Definition: Prevention of degradation of RNA molecules. Subtypes: tRNA stabilization [GO:0036416], GO:0048255, GO:0090669 Relationships: is a type of regulation of RNA stability [GO:0043487]; is_a negative regulation of RNA catabolic process [GO:1902369]